{
  "term_id": "GO:0009986",
  "gene_name": "Interleukin-1 receptor type 1",
  "gene": "UniProtKB:P14778",
  "gene_symbol": "IL1R1",
  "term_label": "cell surface"
}